{
  "term_label": "lysosome",
  "gene": "UniProtKB:P06865",
  "term_id": "GO:0005764",
  "gene_symbol": "HEXA",
  "gene_name": "Beta-hexosaminidase subunit alpha"
}